{
  "gene_symbol": "CATSPERE",
  "term_label": "Unknown molecular function",
  "gene": "UniProtKB:Q5SY80",
  "term_id": "UNKNOWN:0001",
  "gene_name": "Cation channel sperm-associated auxiliary subunit epsilon"
}